{
  "gene": "UniProtKB:P68106",
  "gene_symbol": "FKBP1B",
  "gene_name": "Peptidyl-prolyl cis-trans isomerase FKBP1B",
  "term_label": "protein folding",
  "term_id": "GO:0006457"
}